{
  "gene_name": "Olfactory receptor 5A1",
  "term_id": "GO:0004984",
  "gene": "UniProtKB:Q8NGJ0",
  "term_label": "olfactory receptor activity",
  "gene_symbol": "OR5A1"
}